{
  "gene": "UniProtKB:Q8TAQ9",
  "gene_symbol": "SUN3",
  "term_label": "meiotic nuclear membrane microtubule tethering complex",
  "term_id": "GO:0034993",
  "gene_name": "SUN domain-containing protein 3"
}